{
  "gene_symbol": "EIF2A",
  "gene": "UniProtKB:Q9BY44",
  "gene_name": "Eukaryotic translation initiation factor 2A",
  "term_label": "translational initiation",
  "term_id": "GO:0006413"
}